{
  "term_id": "UNKNOWN:0003",
  "term_label": "Unknown cellular component",
  "gene_name": "Zinc finger protein 281",
  "gene": "UniProtKB:Q9Y2X9",
  "gene_symbol": "ZNF281"
}